root hair cell tip growth [GO:0048768] (biological process) Definition: Localized growth of a plant root hair tip by extension of the cell wall. Also known as: root hair tip growth Relationships: is a type of GO:0009932; is part of root hair elongation [GO:0048767] References: PMID:12468740 Sources: GOC:jid, GOC:ki